{
  "term_label": "plasma membrane",
  "gene_symbol": "PCDHGB7",
  "term_id": "GO:0005886",
  "gene_name": "Protocadherin gamma-B7",
  "gene": "UniProtKB:Q9Y5F8"
}